minus-end-directed organelle transport along microtubule [GO:0072385] (biological process) Relationships: is a type of organelle transport along microtubule [GO:0072384] Sources: GOC:BHF, GOC:mah Also known as: microtubule minus-end-directed organelle localization, microtubule minus-end-directed organelle distribution Subtypes: GO:0072382 Definition: The directed movement of an organelle towards the minus end of a microtubule, mediated by motor proteins. This process begins with the attachment of an organelle to a microtubule, and ends when the organelle reaches its final destination.